{
  "gene": "UniProtKB:Q06141",
  "gene_symbol": "REG3A",
  "term_id": "GO:0008083",
  "term_label": "growth factor activity",
  "gene_name": "Regenerating islet-derived protein 3-alpha"
}